{
  "gene_symbol": "CLDN18",
  "term_id": "GO:0120192",
  "gene": "UniProtKB:P56856",
  "gene_name": "Claudin-18",
  "term_label": "tight junction assembly"
}